{
  "gene_symbol": "RAC2",
  "term_id": "GO:1902622",
  "gene_name": "Ras-related C3 botulinum toxin substrate 2",
  "gene": "UniProtKB:P15153",
  "term_label": "regulation of neutrophil migration"
}